lactam biosynthetic process [GO:0072339] (biological process) Relationships: is a type of amide biosynthetic process [GO:0043604]; is a type of lactam metabolic process [GO:0072338] Also known as: cellular lactam anabolism, cellular lactam biosynthesis, cellular lactam biosynthetic process, cellular lactam formation, cellular lactam synthesis Sources: GOC:mah Subtypes: beta-lactam antibiotic biosynthetic process [GO:0030654], clavulanic acid biosynthetic process [GO:0033050], ansamycin biosynthetic process [GO:0033070], enniatin biosynthetic process [GO:0046585], emericellamide biosynthetic process [GO:1900557], pseurotin A biosynthetic process [GO:1900790] Definition: The chemical reactions and pathways resulting in the formation of lactams, any cyclic amides of amino carboxylic acids, having a 1-azacycloalkan-2-one structure, or analogues having unsaturation or heteroatoms replacing one or more carbon atoms of the ring.